helical viral capsid [GO:0019029] (cellular component) Definition: The protein coat that surrounds the infective nucleic acid in some virus particles; the subunits are arranged to form a protein helix with the genetic material contained within. Tobacco mosaic virus has such a capsid structure. Sources: ISBN:071673706X, UniProtKB-KW:KW-1139, VZ:885 Relationships: is a type of viral capsid [GO:0019028]